protein tyrosine phosphatase complex [GO:1904096] (cellular component) Note: An example of this is ACPP in human (UniProt symbol P15309) in PMID:22389722 (inferred from physical interaction). Relationships: is_a GO:1903293 References: PMID:22389722 Sources: GOC:TermGenie, GOC:bhm, GO_REF:0000088 Definition: A protein complex which is capable of protein tyrosine phosphatase activity.